{
  "term_label": "plasma membrane",
  "term_id": "GO:0005886",
  "gene": "UniProtKB:P43629",
  "gene_symbol": "KIR3DL1",
  "gene_name": "Killer cell immunoglobulin-like receptor 3DL1"
}